regulation of oocyte development [GO:0060281] (BP) Relationships: is a type of regulation of oogenesis [GO:1905879]; regulates oocyte development [GO:0048599] Definition: Any process that modulates the rate or extent of the process whose specific outcome is the progression of an oocyte over time, from initial commitment of the cell to its specific fate, to the fully functional differentiated cell. Subtypes: positive regulation of oocyte development [GO:0060282], GO:0060283 References: PMID:2394318 Sources: GOC:dph, GOC:tb